{
  "term_label": "ruffle membrane",
  "term_id": "GO:0032587",
  "gene_symbol": "ARHGEF2",
  "gene_name": "Rho guanine nucleotide exchange factor 2",
  "gene": "UniProtKB:Q92974"
}